{
  "gene_symbol": "ZNF460",
  "gene_name": "Zinc finger protein 460",
  "gene": "UniProtKB:Q14592",
  "term_label": "RNA polymerase II cis-regulatory region sequence-specific DNA binding",
  "term_id": "GO:0000978"
}